stilbene biosynthetic process [GO:0009811] (biological process) Definition: The chemical reactions and pathways resulting in the formation of stilbenes, a class of polyketide compounds formed from cinnamic acid and three molecules of malonyl CoA. Sources: GOC:tair_curators, ISBN:3110116251 Also known as: stilbene anabolism, stilbene biosynthesis, stilbene formation, stilbene synthesis Relationships: is a type of benzene-containing compound metabolic process [GO:0042537]; is a type of olefinic compound biosynthetic process [GO:0120255]